{
  "term_label": "nucleolus",
  "gene": "UniProtKB:Q8NCV1",
  "gene_name": "Adenosine deaminase domain-containing protein 2",
  "gene_symbol": "ADAD2",
  "term_id": "GO:0005730"
}